S-ribosylhomocysteine lyase activity [GO:0043768] (molecular function) Also known as: S-ribosylhomocysteinase activity, ribosylhomocysteinase activity, LuxS, S-(5-deoxy-D-ribos-5-yl)-L-homocysteine homocysteine-lyase [(4S)-4,5-dihydroxypentan-2,3-dione-forming] Relationships: is a type of carbon-sulfur lyase activity [GO:0016846] Sources: RHEA:17753 Definition: Catalysis of the reaction: S-(5-deoxy-D-ribos-5-yl)-L-homocysteine = (S)-4,5-dihydroxypentane-2,3-dione + L-homocysteine.